trithionate hydrolase activity [GO:0047401] (molecular function) Also known as: trithionate thiosulfohydrolase activity Definition: Catalysis of the reaction: H2O + trithionate = H+ + sulfate + thiosulfate. Relationships: is a type of hydrolase activity, acting on acid sulfur-sulfur bonds [GO:0016828] Sources: RHEA:21884